{
  "term_label": "cartilage development",
  "gene_symbol": "COL11A2",
  "term_id": "GO:0051216",
  "gene_name": "Collagen alpha-2(XI) chain",
  "gene": "UniProtKB:P13942"
}